jasmonyl-Ile conjugate hydrolase activity [GO:1990206] (molecular function) Also known as: JA-Ile hydrolase Definition: Catalysis of the reaction: jasmonyl-Ile + H2O = jasmonic acid + L-isoleucine. Relationships: is a type of hydrolase activity, acting on carbon-nitrogen (but not peptide) bonds [GO:0016810] References: PMID:23943861